{
  "term_id": "GO:0140627",
  "gene_name": "Cullin-2",
  "term_label": "ubiquitin-dependent protein catabolic process via the C-end degron rule pathway",
  "gene": "UniProtKB:Q13617",
  "gene_symbol": "CUL2"
}